{
  "gene": "UniProtKB:Q92621",
  "term_label": "nuclear pore inner ring",
  "term_id": "GO:0044611",
  "gene_name": "Nuclear pore complex protein Nup205",
  "gene_symbol": "NUP205"
}